positive regulation of cell population proliferation [GO:0008284] (BP) Definition: Any process that activates or increases the rate or extent of cell proliferation. Also known as: up regulation of cell proliferation, up-regulation of cell proliferation, upregulation of cell proliferation, activation of cell proliferation, stimulation of cell proliferation, positive regulation of cell proliferation Sources: GOC:go_curators Subtypes: positive regulation of mesenchymal cell proliferation [GO:0002053], positive regulation of skeletal muscle cell proliferation [GO:0014858], positive regulation of osteoblast proliferation [GO:0033690], positive regulation of hemocyte proliferation [GO:0035208], positive regulation of cell proliferation by VEGF-activated platelet derived growth factor receptor signaling pathway [GO:0038091], GO:0048146, GO:0048661, positive regulation of epithelial cell proliferation [GO:0050679], positive regulation of cardiac muscle cell proliferation [GO:0060045], positive regulation of glial cell proliferation [GO:0060252], positive regulation of growth plate cartilage chondrocyte proliferation [GO:0061913], positive regulation of fat cell proliferation [GO:0070346], positive regulation of leukocyte proliferation [GO:0070665], GO:0071338, positive regulation of cell proliferation in bone marrow [GO:0071864], positive regulation of secondary heart field cardioblast proliferation [GO:0072513], GO:1901384, GO:1901724, positive regulation of chondrocyte proliferation [GO:1902732], positive regulation of trophectodermal cell proliferation [GO:1904075], positive regulation of germ cell proliferation [GO:1905938], positive regulation of mammary stem cell proliferation [GO:2000103], positive regulation of cell proliferation involved in heart morphogenesis [GO:2000138], GO:2000179, positive regulation of myoblast proliferation [GO:2000288], positive regulation of cell proliferation involved in compound eye morphogenesis [GO:2000497], positive regulation of stem cell proliferation [GO:2000648] Relationships: is a type of regulation of cell population proliferation [GO:0042127]; is a type of positive regulation of cellular process [GO:0048522]; positively regulates cell population proliferation [GO:0008283]